BRCA2-BRAF35 complex [GO:0002111] (cellular component) Definition: A heterodimeric complex of BRCA2 and BRAF35 (BRCA2-associated factor 35). The BRCA2-BRAF35 complex is often associated with condensed chromatin during mitosis. References: PMID:11207365 Sources: GOC:hjd Relationships: is a type of nuclear protein-containing complex [GO:0140513]